{
  "term_label": "Unknown cellular component",
  "term_id": "UNKNOWN:0003",
  "gene_name": "Olfactory receptor 5AN1",
  "gene_symbol": "OR5AN1",
  "gene": "UniProtKB:Q8NGI8"
}